{
  "gene_name": "FAM231A_C-like protein LOC102723383",
  "gene": "UniProtKB:P0DMU3",
  "gene_symbol": "P0DMU3",
  "term_id": "UNKNOWN:0002",
  "term_label": "Unknown biological process"
}